{
  "gene": "UniProtKB:P40424",
  "gene_name": "Pre-B-cell leukemia transcription factor 1",
  "term_id": "GO:0007420",
  "gene_symbol": "PBX1",
  "term_label": "brain development"
}